{
  "term_label": "positive regulation of synapse assembly",
  "gene_name": "Leucine-rich repeat transmembrane neuronal protein 3",
  "gene": "UniProtKB:Q86VH5",
  "term_id": "GO:0051965",
  "gene_symbol": "LRRTM3"
}